{
  "term_id": "GO:0005886",
  "gene": "UniProtKB:A0PJK1",
  "term_label": "plasma membrane",
  "gene_name": "Sodium_mannose cotransporter SLC5A10",
  "gene_symbol": "SLC5A10"
}